{
  "term_label": "Unknown biological process",
  "gene": "UniProtKB:Q9NQ31",
  "gene_symbol": "AKIP1",
  "term_id": "UNKNOWN:0002",
  "gene_name": "A-kinase-interacting protein 1"
}